{
  "gene": "UniProtKB:Q9H7C4",
  "gene_symbol": "SYNC",
  "term_label": "Z disc",
  "gene_name": "Syncoilin",
  "term_id": "GO:0030018"
}